{
  "gene_symbol": "CPLX2",
  "gene_name": "Complexin-2",
  "term_label": "modulation of chemical synaptic transmission",
  "term_id": "GO:0050804",
  "gene": "UniProtKB:Q6PUV4"
}